{
  "gene_symbol": "SLAMF6",
  "gene": "UniProtKB:Q96DU3",
  "gene_name": "SLAM family member 6",
  "term_label": "T cell activation",
  "term_id": "GO:0042110"
}